{
  "gene": "UniProtKB:Q8IZN3",
  "gene_name": "Palmitoyltransferase ZDHHC14",
  "term_label": "endoplasmic reticulum",
  "term_id": "GO:0005783",
  "gene_symbol": "ZDHHC14"
}